{
  "gene_symbol": "CCNQ",
  "term_id": "GO:0005634",
  "gene_name": "Cyclin-Q",
  "gene": "UniProtKB:Q8N1B3",
  "term_label": "nucleus"
}